positive regulation of intracellular sterol transport [GO:0032382] (biological process) Sources: GOC:mah Definition: Any process that activates or increases the frequency, rate or extent of the directed movement of sterols within cells. Relationships: is a type of positive regulation of sterol transport [GO:0032373]; is a type of positive regulation of intracellular lipid transport [GO:0032379]; is a type of regulation of intracellular sterol transport [GO:0032380]; positively regulates GO:0032366 Also known as: up regulation of intracellular sterol transport, up-regulation of intracellular sterol transport, upregulation of intracellular sterol transport, activation of intracellular sterol transport, stimulation of intracellular sterol transport Subtypes: positive regulation of intracellular cholesterol transport [GO:0032385]